{
  "gene_symbol": "H1-9P",
  "term_id": "GO:0030261",
  "gene_name": "Putative spermatid-specific linker histone H1-like protein",
  "term_label": "chromosome condensation",
  "gene": "UniProtKB:P60008"
}